{
  "gene": "UniProtKB:Q8N5K1",
  "term_label": "mitochondrial outer membrane",
  "gene_symbol": "CISD2",
  "term_id": "GO:0005741",
  "gene_name": "CDGSH iron-sulfur domain-containing protein 2"
}